host cell nuclear matrix [GO:0044204] (cellular component) Sources: GOC:jl, GOC:rynl Relationships: is a type of GO:0044094 Definition: A dynamic, proteinaceous framework within the nucleus of host eukaryotic cells, composed of proteins and RNA, that provides structural support for chromatin organization, gene regulation, and nuclear processes.